{
  "term_label": "Golgi apparatus",
  "gene_symbol": "C11orf24",
  "gene": "UniProtKB:Q96F05",
  "term_id": "GO:0005794",
  "gene_name": "Uncharacterized protein C11orf24"
}